{
  "gene_name": "Neurochondrin",
  "term_id": "GO:0031175",
  "gene_symbol": "NCDN",
  "term_label": "neuron projection development",
  "gene": "UniProtKB:Q9UBB6"
}